{
  "gene_symbol": "RPTOR",
  "term_label": "cellular response to amino acid stimulus",
  "gene_name": "Regulatory-associated protein of mTOR",
  "term_id": "GO:0071230",
  "gene": "UniProtKB:Q8N122"
}